{
  "term_id": "GO:0008408",
  "gene_symbol": "TRIR",
  "gene": "UniProtKB:Q9BQ61",
  "term_label": "3'-5' exonuclease activity",
  "gene_name": "Telomerase RNA component interacting RNase"
}